{
  "term_id": "GO:0007193",
  "gene": "UniProtKB:P07602",
  "term_label": "adenylate cyclase-inhibiting G protein-coupled receptor signaling pathway",
  "gene_symbol": "PSAP",
  "gene_name": "Prosaposin"
}